{
  "gene": "UniProtKB:Q9UFP1",
  "gene_symbol": "GASK1A",
  "gene_name": "Golgi-associated kinase 1A",
  "term_id": "GO:0005794",
  "term_label": "Golgi apparatus"
}